{
  "term_id": "GO:0003723",
  "term_label": "RNA binding",
  "gene_symbol": "DARS1",
  "gene": "UniProtKB:P14868",
  "gene_name": "Aspartate--tRNA ligase, cytoplasmic"
}